{
  "gene_symbol": "ZNF436-AS1",
  "gene_name": "Putative uncharacterized protein ZNF436-AS1",
  "gene": "UniProtKB:Q8NC38",
  "term_id": "UNKNOWN:0003",
  "term_label": "Unknown cellular component"
}